{
  "gene_name": "Lysophosphatidic acid receptor 1",
  "term_id": "GO:0005737",
  "gene_symbol": "LPAR1",
  "term_label": "cytoplasm",
  "gene": "UniProtKB:Q92633"
}